{
  "gene_symbol": "HOMER2",
  "term_id": "GO:0014069",
  "gene": "UniProtKB:Q9NSB8",
  "gene_name": "Homer protein homolog 2",
  "term_label": "postsynaptic density"
}